{
  "term_id": "UNKNOWN:0001",
  "term_label": "Unknown molecular function",
  "gene_symbol": "OMP",
  "gene": "UniProtKB:P47874",
  "gene_name": "Olfactory marker protein"
}